GPI-anchor transamidase activity [GO:0003923] (molecular function) Definition: Catalysis of the formation of the linkage between a protein and a glycosylphosphatidylinositol anchor. The reaction probably occurs by subjecting a peptide bond to nucleophilic attack by the amino group of ethanolamine-GPI, transferring the protein from a signal peptide to the GPI anchor. Sources: ISBN:0471331309 Relationships: is a type of cysteine-type endopeptidase activity [GO:0004197]; is a type of transferase activity, transferring nitrogenous groups [GO:0016769]